{
  "gene_symbol": "GTSF1L",
  "term_id": "UNKNOWN:0001",
  "gene_name": "Gametocyte-specific factor 1-like",
  "term_label": "Unknown molecular function",
  "gene": "UniProtKB:Q9H1H1"
}